{
  "gene": "UniProtKB:Q9UL51",
  "term_id": "GO:0005249",
  "gene_name": "Potassium_sodium hyperpolarization-activated cyclic nucleotide-gated channel 2",
  "term_label": "voltage-gated potassium channel activity",
  "gene_symbol": "HCN2"
}